{
  "gene": "UniProtKB:Q53HC9",
  "term_label": "protein ubiquitination",
  "gene_symbol": "EIPR1",
  "gene_name": "EARP and GARP complex-interacting protein 1",
  "term_id": "GO:0016567"
}